{
  "gene_name": "Ran guanine nucleotide release factor",
  "term_id": "GO:0017080",
  "gene_symbol": "RANGRF",
  "gene": "UniProtKB:Q9HD47",
  "term_label": "sodium channel regulator activity"
}